sperm displacement [GO:0007321] (biological process) Relationships: is a type of sperm competition [GO:0046692] References: PMID:10440373 Definition: The physical displacement of sperm stored from previous mating encounters.